{
  "term_label": "Unknown cellular component",
  "gene": "UniProtKB:A0A075B6W9",
  "term_id": "UNKNOWN:0003",
  "gene_name": "T cell receptor alpha joining 53 (Fragment)",
  "gene_symbol": "TRAJ53"
}